{
  "gene": "UniProtKB:Q99731",
  "term_id": "GO:0006954",
  "term_label": "inflammatory response",
  "gene_name": "C-C motif chemokine 19",
  "gene_symbol": "CCL19"
}